{
  "term_label": "Unknown cellular component",
  "term_id": "UNKNOWN:0003",
  "gene_name": "Cancer_testis antigen family 45 member A3",
  "gene_symbol": "CT45A3",
  "gene": "UniProtKB:Q8NHU0"
}